{
  "gene_name": "Pentraxin-related protein PTX3",
  "term_label": "innate immune response",
  "gene": "UniProtKB:P26022",
  "gene_symbol": "PTX3",
  "term_id": "GO:0045087"
}